{
  "term_id": "GO:0097629",
  "gene": "UniProtKB:Q6ZNE5",
  "gene_name": "Beclin 1-associated autophagy-related key regulator",
  "term_label": "extrinsic component of omegasome membrane",
  "gene_symbol": "ATG14"
}